{
  "gene": "UniProtKB:P61201",
  "term_id": "UNKNOWN:0001",
  "term_label": "Unknown molecular function",
  "gene_symbol": "COPS2",
  "gene_name": "COP9 signalosome complex subunit 2"
}